{
  "gene_symbol": "ZNF594",
  "gene": "UniProtKB:Q96JF6",
  "term_label": "transcription cis-regulatory region binding",
  "term_id": "GO:0000976",
  "gene_name": "Zinc finger protein 594"
}